{
  "term_id": "GO:0007189",
  "gene_name": "Adenylate cyclase type 6",
  "term_label": "adenylate cyclase-activating G protein-coupled receptor signaling pathway",
  "gene": "UniProtKB:O43306",
  "gene_symbol": "ADCY6"
}